{
  "gene_symbol": "MRTO4",
  "gene_name": "mRNA turnover protein 4 homolog",
  "gene": "UniProtKB:Q9UKD2",
  "term_label": "nuclear-transcribed mRNA catabolic process",
  "term_id": "GO:0000956"
}